{
  "term_id": "GO:0005886",
  "gene": "UniProtKB:Q8NH61",
  "gene_name": "Olfactory receptor 51F2",
  "term_label": "plasma membrane",
  "gene_symbol": "OR51F2"
}